{
  "term_label": "CAAX-box protein processing",
  "gene": "UniProtKB:O75844",
  "gene_symbol": "ZMPSTE24",
  "term_id": "GO:0071586",
  "gene_name": "CAAX prenyl protease 1 homolog"
}